Gtr1-Gtr2 GTPase complex [GO:1990131] (CC) Definition: A heterodimer GTPase complex. In S. cerevisiae, this complex contains Gtr1p and Gtr2p proteins. Relationships: is a type of GTPase complex [GO:1905360] References: PMID:10388807, PMID:16143306 Sources: GOC:rb